{
  "gene": "UniProtKB:P02778",
  "gene_symbol": "CXCL10",
  "term_label": "extracellular space",
  "gene_name": "C-X-C motif chemokine 10",
  "term_id": "GO:0005615"
}